{
  "gene_symbol": "TMEM158",
  "gene_name": "Transmembrane protein 158",
  "term_id": "UNKNOWN:0002",
  "term_label": "Unknown biological process",
  "gene": "UniProtKB:Q8WZ71"
}